{
  "term_id": "GO:0005829",
  "term_label": "cytosol",
  "gene_symbol": "IFIT2",
  "gene": "UniProtKB:P09913",
  "gene_name": "Interferon-induced protein with tetratricopeptide repeats 2"
}